{
  "term_label": "regulation of intracellular signal transduction",
  "gene": "UniProtKB:Q96PV0",
  "gene_symbol": "SYNGAP1",
  "term_id": "GO:1902531",
  "gene_name": "Ras_Rap GTPase-activating protein SynGAP"
}